{
  "gene": "UniProtKB:P68032",
  "gene_name": "Actin, alpha cardiac muscle 1",
  "term_id": "GO:0015629",
  "term_label": "actin cytoskeleton",
  "gene_symbol": "ACTC1"
}